{
  "term_label": "rRNA binding",
  "gene_name": "Large ribosomal subunit protein uL16m",
  "gene_symbol": "MRPL16",
  "term_id": "GO:0019843",
  "gene": "UniProtKB:Q9NX20"
}